epidermal growth factor receptor signaling pathway involved in heart process [GO:1905251] (biological process) Also known as: EGF receptor signaling pathway involved in heart process, EGF receptor signalling pathway involved in heart process, EGFR signaling pathway involved in heart process, ERBB1 signaling pathway involved in heart process, epidermal growth factor receptor signalling pathway involved in heart process, receptor tyrosine-protein kinase erbB-1 signaling pathway involved in heart process, EGF receptor signaling pathway involved in cardiac process, EGF receptor signalling pathway involved in cardiac process, EGFR signaling pathway involved in cardiac process, ERBB1 signaling pathway involved in cardiac process, epidermal growth factor receptor signaling pathway involved in cardiac process, epidermal growth factor receptor signalling pathway involved in cardiac process, receptor tyrosine-protein kinase erbB-1 signaling pathway involved in cardiac process Regulation: regulated by GO:1905282; negatively regulated by negative regulation of epidermal growth factor receptor signaling pathway involved in heart process [GO:1905283]; positively regulated by positive regulation of epidermal growth factor receptor signaling pathway involved in heart process [GO:1905284] Definition: Any epidermal growth factor receptor signaling pathway that is involved in heart process. Relationships: is a type of epidermal growth factor receptor signaling pathway [GO:0007173]; is part of GO:0003015 References: PMID:23069713 Sources: GOC:BHF, GOC:BHF_miRNA, GOC:TermGenie, GOC:bc, GO_REF:0000060